{
  "gene": "UniProtKB:Q8IZF4",
  "term_id": "GO:0007186",
  "gene_symbol": "ADGRG5",
  "term_label": "G protein-coupled receptor signaling pathway",
  "gene_name": "Adhesion G-protein coupled receptor G5"
}